{
  "term_id": "GO:0005765",
  "gene": "UniProtKB:P01906",
  "gene_name": "HLA class II histocompatibility antigen, DQ alpha 2 chain",
  "gene_symbol": "HLA-DQA2",
  "term_label": "lysosomal membrane"
}